{
  "term_id": "UNKNOWN:0003",
  "gene_symbol": "HAND2",
  "gene_name": "Heart- and neural crest derivatives-expressed protein 2",
  "gene": "UniProtKB:P61296",
  "term_label": "Unknown cellular component"
}